{
  "gene": "UniProtKB:Q2TBA0",
  "gene_name": "Kelch-like protein 40",
  "gene_symbol": "KLHL40",
  "term_label": "I band",
  "term_id": "GO:0031674"
}